{
  "gene_symbol": "DYSF",
  "gene": "UniProtKB:O75923",
  "term_label": "synaptic vesicle membrane",
  "term_id": "GO:0030672",
  "gene_name": "Dysferlin"
}